{
  "gene_name": "Homeobox protein Hox-A9",
  "gene_symbol": "HOXA9",
  "gene": "UniProtKB:P31269",
  "term_label": "nucleus",
  "term_id": "GO:0005634"
}